{
  "gene_name": "E3 ubiquitin-protein ligase MARCHF4",
  "gene": "UniProtKB:Q9P2E8",
  "term_id": "GO:0004842",
  "term_label": "ubiquitin-protein transferase activity",
  "gene_symbol": "MARCHF4"
}